UDP-glucose:glycoprotein glucosyltransferase activity [GO:0003980] (molecular function) Definition: Catalysis of the addition of UDP-glucose on to asparagine-linked (N-linked) oligosaccharides of the form Man7-9GlcNAc2 on incorrectly folded glycoproteins. References: PMID:10764828 Sources: GOC:al Also known as: UGGT activity Relationships: is a type of UDP-glucosyltransferase activity [GO:0035251]; is part of GO:0097359